meiosis I/meiosis II transition [GO:1990946] (biological process) Relationships: is a type of meiotic cell cycle phase transition [GO:0044771] Definition: The cell cycle process in which a cell progresses from meiosis I to meiosis II. References: PMID:21389117